dITP catabolic process [GO:0035863] (biological process) Definition: The chemical reactions and pathways resulting in the breakdown of dITP, a deoxyinosine phosphate compound having a triphosphate group at the 5'-position. Sources: GOC:dgf Also known as: 2'-Deoxyinosine 5'-triphosphate catabolic process, 2'-Deoxyinosine-5'-triphosphate catabolic process, dITP breakdown, dITP catabolism, dITP degradation, deoxyinosine 5'-triphosphate catabolic process, deoxyinosine triphosphate (2'-deoxyinosine 5'-triphosphate) catabolic process Relationships: is a type of GO:0009155; is a type of GO:0009217